{
  "term_id": "GO:0006355",
  "gene_symbol": "ZNF626",
  "term_label": "regulation of DNA-templated transcription",
  "gene": "UniProtKB:Q68DY1",
  "gene_name": "Zinc finger protein 626"
}